GTP-dependent polyribonucleotide 5'-hydroxyl-kinase activity [GO:0051730] (molecular function) Also known as: GTP-dependent RNA 5'-hydroxyl-kinase activity, GTP-dependent RNA kinase activity, GTP-dependent polyribonucleotide kinase activity Definition: Catalysis of the reaction: GTP + 5'-dephospho-RNA = GDP + 5'-phospho-RNA. References: PMID:8428918 Relationships: is a type of GTP-dependent polynucleotide 5'-hydroxyl-kinase activity [GO:0051735]